{
  "gene_name": "Galactosylceramide sulfotransferase",
  "term_label": "galactosylceramide biosynthetic process",
  "gene_symbol": "GAL3ST1",
  "gene": "UniProtKB:Q99999",
  "term_id": "GO:0006682"
}